positive regulation of R8 cell differentiation [GO:0045681] (biological process) Also known as: positive regulation of R8 differentiation, up regulation of R8 differentiation, up-regulation of R8 differentiation, upregulation of R8 differentiation, activation of R8 differentiation, stimulation of R8 differentiation Sources: GOC:dph, GOC:go_curators, GOC:tb Definition: Any process that activates or increases the frequency, rate or extent of R8 cell differentiation. Relationships: is a type of regulation of R8 cell differentiation [GO:0045679]; is a type of positive regulation of compound eye photoreceptor cell differentiation [GO:0110117]; positively regulates R8 cell differentiation [GO:0045465]